{
  "term_label": "Unknown molecular function",
  "term_id": "UNKNOWN:0001",
  "gene_name": "T cell receptor alpha joining 30 (Fragment)",
  "gene_symbol": "TRAJ30",
  "gene": "UniProtKB:A0A075B6Y1"
}